{
  "gene_name": "LYR motif-containing protein 9",
  "term_id": "UNKNOWN:0001",
  "gene": "UniProtKB:A8MSI8",
  "gene_symbol": "LYRM9",
  "term_label": "Unknown molecular function"
}